{
  "term_label": "histone deacetylase binding",
  "gene": "UniProtKB:Q02080",
  "gene_symbol": "MEF2B",
  "term_id": "GO:0042826",
  "gene_name": "Myocyte-specific enhancer factor 2B"
}